glutathione-CoA-glutathione transhydrogenase activity [GO:0047140] (molecular function) Relationships: is a type of oxidoreductase activity, acting on a sulfur group of donors, disulfide as acceptor [GO:0016671] Sources: EC:1.8.4.3, MetaCyc:1.8.4.3-RXN Definition: Catalysis of the reaction: oxidized glutathione + CoA = reduced glutathione + CoA-glutathione. Also known as: CoA:glutathione-disulfide oxidoreductase activity, coenzyme A:glutathione-disulfide oxidoreductase activity, coenzyme A:oxidized-glutathione oxidoreductase activity, glutathione coenzyme A-glutathione transhydrogenase activity, glutathione-coenzyme A glutathione disulfide transhydrogenase activity, glutathione:coenzyme A-glutathione transhydrogenase activity